{
  "gene": "UniProtKB:Q8NCN5",
  "gene_name": "Pyruvate dehydrogenase phosphatase regulatory subunit, mitochondrial",
  "gene_symbol": "PDPR",
  "term_id": "GO:0005759",
  "term_label": "mitochondrial matrix"
}